{
  "gene_symbol": "RING1",
  "gene_name": "E3 ubiquitin-protein ligase RING1",
  "term_label": "negative regulation of DNA-templated transcription",
  "gene": "UniProtKB:Q06587",
  "term_id": "GO:0045892"
}